{
  "gene_symbol": "HSPA1B",
  "term_id": "GO:0032436",
  "gene_name": "Heat shock 70 kDa protein 1B",
  "gene": "UniProtKB:P0DMV9",
  "term_label": "positive regulation of proteasomal ubiquitin-dependent protein catabolic process"
}